tyrosine-tRNA ligase activity [GO:0004831] (molecular function) Relationships: is a type of aminoacyl-tRNA ligase activity [GO:0004812] Sources: EC:6.1.1.1, RHEA:10220 Definition: Catalysis of the reaction: L-tyrosine + ATP + tRNA(Tyr) = L-tyrosyl-tRNA(Tyr) + AMP + diphosphate + 2 H+. Also known as: tyrosyl-tRNA synthetase activity, L-tyrosine-tRNA(Tyr) ligase (AMP-forming) activity, L-tyrosine-tRNATyr ligase (AMP-forming), L-tyrosine:tRNATyr ligase (AMP-forming), tyrosine tRNA synthetase activity, tyrosine translase activity, tyrosine-transfer RNA ligase activity, tyrosine-transfer ribonucleate synthetase activity, tyrosyl-tRNA ligase activity, tyrosyl-transfer RNA synthetase activity, tyrosyl-transfer ribonucleate synthetase activity, tyrosyl-transfer ribonucleic acid synthetase activity